{
  "gene": "UniProtKB:Q8NEG2",
  "term_id": "UNKNOWN:0002",
  "gene_symbol": "C7orf57",
  "gene_name": "Uncharacterized protein C7orf57",
  "term_label": "Unknown biological process"
}